negative regulation of phospholipase C-activating G protein-coupled receptor signaling pathway [GO:1900737] (biological process) Definition: Any process that stops, prevents or reduces the frequency, rate or extent of phospholipase C-activating G protein-coupled receptor signaling pathway. Subtypes: negative regulation of phospholipase C-activating phototransduction signaling pathway [GO:0016060], negative regulation of phospholipase C-activating dopamine receptor signaling pathway [GO:0060162] Relationships: is_a GO:0045744; is_a regulation of phospholipase C-activating G protein-coupled receptor signaling pathway [GO:1900736]; negatively regulates phospholipase C-activating G protein-coupled receptor signaling pathway [GO:0007200] Sources: GOC:BHF, GOC:TermGenie Also known as: down regulation of G protein signaling, coupled to IP3 second messenger (phospholipase C activating), down regulation of G protein signalling, coupled to IP3 second messenger (phospholipase C activating), down regulation of G-protein coupled receptor signaling pathway coupled to IP3 second messenger, down regulation of G-protein signaling, coupled to IP3 second messenger (phospholipase C activating), down regulation of G-protein signalling, coupled to IP3 second messenger (phospholipase C activating), down regulation of PLC-activating GPCR signaling pathway, down regulation of phospholipase C-activating G-protein coupled receptor signaling pathway, down-regulation of G protein signaling, coupled to IP3 second messenger (phospholipase C activating), down-regulation of G protein signalling, coupled to IP3 second messenger (phospholipase C activating), down-regulation of G-protein coupled receptor signaling pathway coupled to IP3 second messenger, down-regulation of G-protein signaling, coupled to IP3 second messenger (phospholipase C activating), down-regulation of G-protein signalling, coupled to IP3 second messenger (phospholipase C activating), down-regulation of PLC-activating GPCR signaling pathway, down-regulation of phospholipase C-activating G-protein coupled receptor signaling pathway, downregulation of G protein signaling, coupled to IP3 second messenger (phospholipase C activating), downregulation of G protein signalling, coupled to IP3 second messenger (phospholipase C activating), downregulation of G-protein coupled receptor signaling pathway coupled to IP3 second messenger, downregulation of G-protein signaling, coupled to IP3 second messenger (phospholipase C activating), downregulation of G-protein signalling, coupled to IP3 second messenger (phospholipase C activating), downregulation of PLC-activating GPCR signaling pathway, downregulation of phospholipase C-activating G-protein coupled receptor signaling pathway, inhibition of G protein signaling, coupled to IP3 second messenger (phospholipase C activating), inhibition of G protein signalling, coupled to IP3 second messenger (phospholipase C activating), inhibition of G-protein coupled receptor signaling pathway coupled to IP3 second messenger, inhibition of G-protein signaling, coupled to IP3 second messenger (phospholipase C activating), inhibition of G-protein signalling, coupled to IP3 second messenger (phospholipase C activating), inhibition of PLC-activating GPCR signaling pathway, negative regulation of G protein signaling, coupled to IP3 second messenger (phospholipase C activating), negative regulation of G protein signalling, coupled to IP3 second messenger (phospholipase C activating), negative regulation of G-protein coupled receptor signaling pathway coupled to IP3 second messenger, negative regulation of G-protein signaling, coupled to IP3 second messenger (phospholipase C activating), negative regulation of G-protein signalling, coupled to IP3 second messenger (phospholipase C activating), negative regulation of PLC-activating GPCR signaling pathway, negative regulation of phospholipase C-activating G-protein coupled receptor signaling pathway, down regulation of phospholipase C-activating dopamine receptor signaling pathway, down-regulation of phospholipase C-activating dopamine receptor signaling pathway, downregulation of phospholipase C-activating dopamine receptor signaling pathway, inhibition of phospholipase C-activating G-protein coupled receptor signaling pathway, inhibition of phospholipase C-activating dopamine receptor signaling pathway, negative regulation of phospholipase C-activating dopamine receptor signaling pathway, down regulation of activation of phospholipase C activity by G-protein coupled receptor protein signaling pathway coupled to IP3 second messenger, down-regulation of activation of phospholipase C activity by G-protein coupled receptor protein signaling pathway coupled to IP3 second messenger, downregulation of activation of phospholipase C activity by G-protein coupled receptor protein signaling pathway coupled to IP3 second messenger, inhibition of activation of phospholipase C activity by G-protein coupled receptor protein signaling pathway coupled to IP3 second messenger, negative regulation of activation of phospholipase C activity by G-protein coupled receptor protein signaling pathway coupled to IP3 second messenger